{
  "gene_name": "Protein FAM118A",
  "term_label": "Unknown molecular function",
  "term_id": "UNKNOWN:0001",
  "gene": "UniProtKB:Q9NWS6",
  "gene_symbol": "FAM118A"
}